{
  "term_id": "GO:0034599",
  "term_label": "cellular response to oxidative stress",
  "gene_name": "Glutathione peroxidase 2",
  "gene": "UniProtKB:P18283",
  "gene_symbol": "GPX2"
}